{
  "term_id": "GO:0005096",
  "gene_symbol": "RALGAPB",
  "gene_name": "Ral GTPase-activating protein subunit beta",
  "gene": "UniProtKB:Q86X10",
  "term_label": "GTPase activator activity"
}